{
  "gene": "UniProtKB:O60879",
  "term_label": "Unknown molecular function",
  "gene_name": "Protein diaphanous homolog 2",
  "gene_symbol": "DIAPH2",
  "term_id": "UNKNOWN:0001"
}